{
  "term_id": "GO:0005737",
  "gene_symbol": "CDADC1",
  "gene": "UniProtKB:Q9BWV3",
  "term_label": "cytoplasm",
  "gene_name": "Cytidine and dCMP deaminase domain-containing protein 1"
}